cellular response to ammonium ion [GO:0071242] (biological process) Relationships: is a type of response to ammonium ion [GO:0060359]; is a type of cellular response to nitrogen compound [GO:1901699] References: PMID:23509267 Sources: GOC:TermGenie, GO_REF:0000071 Also known as: cellular response to ammonia Definition: Any process that results in a change in state or activity of a cell (in terms of movement, secretion, enzyme production, gene expression, etc.) as a result of an ammonium stimulus.